{
  "gene_symbol": "OR1D5",
  "gene": "UniProtKB:P58170",
  "gene_name": "Olfactory receptor 1D5",
  "term_label": "signal transduction",
  "term_id": "GO:0007165"
}